{
  "term_label": "N-acetylglucosamine metabolic process",
  "gene_name": "Carbohydrate sulfotransferase 3",
  "gene": "UniProtKB:Q7LGC8",
  "term_id": "GO:0006044",
  "gene_symbol": "CHST3"
}